naphtho-gamma-pyrone catabolic process [GO:1900786] (BP) Also known as: naphtho-gamma-pyrone breakdown, naphtho-gamma-pyrone catabolism, naphtho-gamma-pyrone degradation, naphtho-gamma-pyrones breakdown, naphtho-gamma-pyrones catabolic process, naphtho-gamma-pyrones catabolism, naphtho-gamma-pyrones degradation Definition: The chemical reactions and pathways resulting in the breakdown of naphtho-gamma-pyrone. Subtypes: fonsecin catabolic process [GO:1900768] Sources: GOC:TermGenie, GOC:di Relationships: is a type of ketone catabolic process [GO:0042182]